{
  "gene_symbol": "DNAH8",
  "term_id": "GO:0036158",
  "gene_name": "Dynein axonemal heavy chain 8",
  "term_label": "outer dynein arm assembly",
  "gene": "UniProtKB:Q96JB1"
}